{
  "gene": "UniProtKB:Q96EH8",
  "term_id": "GO:0061630",
  "gene_name": "E3 ubiquitin-protein ligase NEURL3",
  "gene_symbol": "NEURL3",
  "term_label": "ubiquitin protein ligase activity"
}